{
  "gene": "UniProtKB:P81277",
  "term_label": "response to peptide hormone",
  "gene_name": "Prolactin-releasing peptide",
  "gene_symbol": "PRLH",
  "term_id": "GO:0043434"
}